{
  "gene_name": "Cysteine--tRNA ligase, cytoplasmic",
  "term_label": "cysteinyl-tRNA aminoacylation",
  "term_id": "GO:0006423",
  "gene_symbol": "CARS1",
  "gene": "UniProtKB:P49589"
}